{
  "term_label": "U2-type catalytic step 1 spliceosome",
  "gene": "UniProtKB:Q9NW64",
  "term_id": "GO:0071006",
  "gene_symbol": "RBM22",
  "gene_name": "Pre-mRNA-splicing factor RBM22"
}